{
  "term_label": "male gonad development",
  "gene_name": "3-oxo-5-alpha-steroid 4-dehydrogenase 1",
  "gene": "UniProtKB:P18405",
  "term_id": "GO:0008584",
  "gene_symbol": "SRD5A1"
}